{
  "term_id": "GO:0032266",
  "gene": "UniProtKB:Q68DK2",
  "gene_name": "Zinc finger FYVE domain-containing protein 26",
  "gene_symbol": "ZFYVE26",
  "term_label": "phosphatidylinositol-3-phosphate binding"
}